defense response to bacterium [GO:0042742] (biological process) Sources: GOC:jl Subtypes: induced systemic resistance [GO:0009682], antibacterial humoral response [GO:0019731], GO:0050829, defense response to Gram-positive bacterium [GO:0050830], male-specific defense response to bacterium [GO:0050831], GO:0140367 Also known as: defence response to bacteria, defence response to bacterium, defense response to bacteria, defense response to bacterium, incompatible interaction, resistance response to pathogenic bacteria, resistance response to pathogenic bacterium, antibacterial peptide activity Relationships: is a type of GO:0006952; is a type of GO:0009617 Regulation: regulated by regulation of defense response to bacterium [GO:1900424]; negatively regulated by GO:1900425; positively regulated by positive regulation of defense response to bacterium [GO:1900426] Definition: Reactions triggered in response to the presence of a bacterium that act to protect the cell or organism.